{
  "term_id": "UNKNOWN:0003",
  "term_label": "Unknown cellular component",
  "gene_name": "Transmembrane protein 215",
  "gene": "UniProtKB:Q68D42",
  "gene_symbol": "TMEM215"
}